auxin catabolic process [GO:0009852] (biological process) Relationships: is a type of auxin metabolic process [GO:0009850]; is a type of hormone catabolic process [GO:0042447] Subtypes: GO:0042437 Sources: GOC:lm, GOC:lr, ISBN:0198547684 Also known as: auxin breakdown, auxin catabolism, auxin degradation Definition: The chemical reactions and pathways resulting in the breakdown of auxins, a group of plant hormones that regulate aspects of plant growth.